{
  "gene_symbol": "JAKMIP2",
  "gene_name": "Janus kinase and microtubule-interacting protein 2",
  "term_id": "UNKNOWN:0003",
  "gene": "UniProtKB:Q96AA8",
  "term_label": "Unknown cellular component"
}